{
  "gene_symbol": "TMEM230",
  "term_label": "Unknown molecular function",
  "gene": "UniProtKB:Q96A57",
  "term_id": "UNKNOWN:0001",
  "gene_name": "Transmembrane protein 230"
}